{
  "gene": "UniProtKB:Q9H3D4",
  "gene_symbol": "TP63",
  "term_id": "GO:0005634",
  "term_label": "nucleus",
  "gene_name": "Tumor protein 63"
}